{
  "term_id": "GO:0005737",
  "gene_name": "Prefoldin subunit 2",
  "gene_symbol": "PFDN2",
  "term_label": "cytoplasm",
  "gene": "UniProtKB:Q9UHV9"
}